positive regulation of purine nucleotide catabolic process [GO:0033123] (BP) Subtypes: GO:0045821 Sources: GOC:mah Definition: Any process that activates or increases the frequency, rate or extent of the chemical reactions and pathways resulting in the breakdown of purine nucleotides. Also known as: positive regulation of purine nucleotide breakdown, positive regulation of purine nucleotide catabolism, positive regulation of purine nucleotide degradation Relationships: is a type of positive regulation of nucleotide catabolic process [GO:0030813]; is a type of GO:0033121; is a type of positive regulation of purine nucleotide metabolic process [GO:1900544]; positively regulates GO:0006195